acetylcholine secretion, neurotransmission [GO:0014055] (biological process) Relationships: is a type of neurotransmitter secretion [GO:0007269]; is a type of acetylcholine secretion [GO:0061526]; is part of synaptic transmission, cholinergic [GO:0007271] Definition: The regulated release of acetylcholine by a cell. The acetylcholine acts as a neurotransmitter that acts in both the peripheral nervous system (PNS) and central nervous system (CNS). Regulation: regulated by regulation of acetylcholine secretion, neurotransmission [GO:0014056]; positively regulated by GO:0014057; negatively regulated by negative regulation of acetylcholine secretion, neurotransmission [GO:0014058] Sources: GOC:ef